{
  "term_id": "GO:0070037",
  "gene": "UniProtKB:Q92979",
  "gene_name": "Ribosomal RNA small subunit methyltransferase NEP1",
  "term_label": "rRNA (pseudouridine) methyltransferase activity",
  "gene_symbol": "EMG1"
}